{
  "gene_name": "Elongation of very long chain fatty acids protein 5",
  "gene_symbol": "ELOVL5",
  "term_label": "fatty acid elongation, monounsaturated fatty acid",
  "gene": "UniProtKB:Q9NYP7",
  "term_id": "GO:0034625"
}